positive regulation of signal transduction [GO:0009967] (biological process) Subtypes: positive regulation of cytokine-mediated signaling pathway [GO:0001961], GO:0009789, positive regulation of gibberellic acid mediated signaling pathway [GO:0009939], positive regulation of platelet-derived growth factor receptor signaling pathway [GO:0010641], positive regulation of auxin mediated signaling pathway [GO:0010929], positive adaptation of signaling pathway [GO:0023059], positive regulation of Wnt signaling pathway [GO:0030177], positive regulation of vascular endothelial growth factor receptor signaling pathway [GO:0030949], positive regulation of brain-derived neurotrophic factor receptor signaling pathway [GO:0031550], positive regulation of lipopolysaccharide-mediated signaling pathway [GO:0031666], GO:0035388, positive regulation of signal transduction by receptor internalization [GO:0038010], positive regulation of insulin-like growth factor receptor signaling pathway [GO:0043568], positive regulation of fibroblast growth factor receptor signaling pathway [GO:0045743], positive regulation of G protein-coupled receptor signaling pathway [GO:0045745], GO:0045747, positive regulation of Toll signaling pathway [GO:0045752], GO:0045874, positive regulation of smoothened signaling pathway [GO:0045880], positive regulation of insulin receptor signaling pathway [GO:0046628], positive regulation of antigen receptor-mediated signaling pathway [GO:0050857], positive regulation of neurotrophin TRK receptor signaling pathway [GO:0051388], positive regulation of signal transduction involved in conjugation with cellular fusion [GO:0060239], GO:0060369, positive regulation of growth hormone receptor signaling pathway [GO:0060399], GO:0062208, GO:0080038, positive regulation of salicylic acid mediated signaling pathway [GO:0080151], GO:0090100, GO:0090228, positive regulation of torso signaling pathway [GO:0120176], positive regulation of glutamate receptor signaling pathway [GO:1900451], positive regulation of brassinosteroid mediated signaling pathway [GO:1900459], positive regulation of vascular endothelial growth factor signaling pathway [GO:1900748], positive regulation of ERBB signaling pathway [GO:1901186], positive regulation of ephrin receptor signaling pathway [GO:1901189], positive regulation of Fas signaling pathway [GO:1902046], positive regulation of sphingolipid mediated signaling pathway [GO:1902070], positive regulation of hepatocyte growth factor receptor signaling pathway [GO:1902204], positive regulation of intracellular signal transduction [GO:1902533], positive regulation of glucose mediated signaling pathway [GO:1902661], positive regulation of netrin-activated signaling pathway [GO:1902843], positive regulation of neuronal signal transduction [GO:1902849], positive regulation of receptor signaling pathway via STAT [GO:1904894], positive regulation of apolipoprotein A-I-mediated signaling pathway [GO:1905096], GO:2000350, positive regulation of excitatory postsynaptic potential [GO:2000463], positive regulation of glial cell-derived neurotrophic factor receptor signaling pathway involved in ureteric bud formation [GO:2000735], positive regulation of integrin-mediated signaling pathway [GO:2001046], positive regulation of apoptotic signaling pathway [GO:2001235], positive regulation of semaphorin-plexin signaling pathway [GO:2001262] Sources: GOC:sm Relationships: is a type of regulation of signal transduction [GO:0009966]; is a type of GO:0010647; is a type of GO:0023056; is a type of GO:0048584; positively regulates signal transduction [GO:0007165] Also known as: up regulation of signal transduction, up-regulation of signal transduction, upregulation of signal transduction, activation of signal transduction, stimulation of signal transduction, positive regulation of signaling pathway, positive regulation of signalling pathway Definition: Any process that activates or increases the frequency, rate or extent of signal transduction.